{
  "term_id": "GO:0005737",
  "term_label": "cytoplasm",
  "gene": "UniProtKB:Q9H171",
  "gene_symbol": "ZBP1",
  "gene_name": "Z-DNA-binding protein 1"
}